{
  "gene_name": "Protein phosphatase 1 regulatory subunit 12B",
  "gene_symbol": "PPP1R12B",
  "term_label": "Z disc",
  "term_id": "GO:0030018",
  "gene": "UniProtKB:O60237"
}